{
  "gene_symbol": "IRAK4",
  "term_id": "GO:0035556",
  "term_label": "intracellular signal transduction",
  "gene": "UniProtKB:Q9NWZ3",
  "gene_name": "Interleukin-1 receptor-associated kinase 4"
}